{
  "term_id": "GO:0000149",
  "gene": "UniProtKB:Q8WVH0",
  "term_label": "SNARE binding",
  "gene_symbol": "CPLX3",
  "gene_name": "Complexin-3"
}